{
  "term_id": "GO:0006915",
  "gene_symbol": "PLSCR3",
  "gene_name": "Phospholipid scramblase 3",
  "term_label": "apoptotic process",
  "gene": "UniProtKB:Q9NRY6"
}